cellular response to red light [GO:0071491] (biological process) Definition: Any process that results in a change in state or activity of a cell (in terms of movement, secretion, enzyme production, gene expression, etc.) as a result of a red light stimulus. Red light is electromagnetic radiation of wavelength of 580-700nm. An example of this response is seen at the beginning of many plant species developmental stages. These include germination, and the point when cotyledon expansion is triggered. In certain species these processes take place in response to absorption of red light by the pigment molecule phytochrome, but the signal can be reversed by exposure to far red light. During the initial phase the phytochrome molecule is only present in the red light absorbing form, but on absorption of red light it changes to a far red light absorbing form, triggering progress through development. An immediate short period of exposure to far red light entirely returns the pigment to its initial state and prevents triggering of the developmental process. A thirty minute break between red and subsequent far red light exposure renders the red light effect irreversible, and development then occurs regardless of whether far red light exposure subsequently occurs. Also known as: cellular response to red light stimulus Subtypes: red light signaling pathway [GO:0010161] Relationships: is a type of response to red light [GO:0010114]; is a type of cellular response to red or far red light [GO:0071489] Sources: GOC:mah